cyclin D3-CDK6 complex [GO:0097133] (cellular component) References: PMID:15935619 Sources: GOC:so Relationships: is a type of cyclin-dependent protein kinase holoenzyme complex [GO:0000307] Definition: A protein complex consisting of cyclin D3 and cyclin-dependent kinase 6 (CDK6). Cyclins are characterized by periodicity in protein abundance throughout the cell cycle. Cyclin-dependent kinases represent a family of serine/threonine protein kinases that become active upon binding to a cyclin regulatory partner.